{
  "gene_name": "Polyunsaturated fatty acid lipoxygenase ALOX15",
  "term_label": "plasma membrane",
  "gene": "UniProtKB:P16050",
  "term_id": "GO:0005886",
  "gene_symbol": "ALOX15"
}